{
  "gene_symbol": "NOTCH4",
  "gene_name": "Neurogenic locus notch homolog protein 4",
  "term_label": "Notch binding",
  "gene": "UniProtKB:Q99466",
  "term_id": "GO:0005112"
}